{
  "term_id": "GO:0005737",
  "gene": "UniProtKB:P25713",
  "term_label": "cytoplasm",
  "gene_symbol": "MT3",
  "gene_name": "Metallothionein-3"
}